{
  "term_id": "UNKNOWN:0002",
  "gene": "UniProtKB:Q8TAV0",
  "term_label": "Unknown biological process",
  "gene_symbol": "FAM76A",
  "gene_name": "Protein FAM76A"
}